{
  "term_label": "nucleus",
  "gene_symbol": "RITA1",
  "term_id": "GO:0005634",
  "gene_name": "RBPJ-interacting and tubulin-associated protein 1",
  "gene": "UniProtKB:Q96K30"
}